{
  "term_id": "GO:0046928",
  "term_label": "regulation of neurotransmitter secretion",
  "gene_name": "Multiple C2 and transmembrane domain-containing protein 1",
  "gene": "UniProtKB:Q6DN14",
  "gene_symbol": "MCTP1"
}